ribose phosphate diphosphokinase complex [GO:0002189] (CC) Note: In mammals, the complex consists of two non-identical catalytic subunits and two non-identical regulatory subunits. Also known as: PRPP synthetase complex, phosphoribosylpyrophosphate synthetase complex References: PMID:9348095 Sources: GO:hjd Relationships: is a type of GO:0061695 Definition: A protein complex having ribose phosphate diphosphokinase activity.